Golgi vesicle fusion with endoplasmic reticulum-Golgi intermediate compartment (ERGIC) membrane [GO:1990688] (biological process) References: PMID:16038056, PMID:24119662 Sources: GOC:bhm Relationships: is a type of vesicle fusion with endoplasmic reticulum-Golgi intermediate compartment (ERGIC) membrane [GO:1990668]; is part of GO:0006890 Also known as: Golgi vesicle fusion with ER-Golgi intermediate compartment membrane, Golgi vesicle fusion with ERGIC membrane Definition: The joining of the lipid bilayer membrane around a Golgi vesicle to the lipid bilayer membrane of the ERGIC. Such vesicles include COPI-coated transport vesicles involved in retrograde transport.